{
  "term_label": "Unknown molecular function",
  "gene": "UniProtKB:Q9UHR6",
  "gene_name": "Zinc finger HIT domain-containing protein 2",
  "gene_symbol": "ZNHIT2",
  "term_id": "UNKNOWN:0001"
}